organelle inner membrane [GO:0019866] (cellular component) Subtypes: GO:0005637, mitochondrial inner membrane [GO:0005743], GO:0009528 Sources: GOC:mah Relationships: is a type of GO:0031090; is part of GO:0031967 Definition: The inner, i.e. lumen-facing, lipid bilayer of an organelle envelope; usually highly selective to most ions and metabolites. Note: See also the cellular component term 'outer membrane ; GO:0019867'.